tRNA queuosine(34) biosynthetic process from salvaged queuine [GO:0160255] (biological process) References: PMID:28208705, PMID:39600051 Sources: MetaCyc:PWY-8105 Relationships: is a type of tRNA queuosine(34) biosynthetic process [GO:0008616] Definition: The chemical reactions and pathways resulting in the formation of tRNA queuosine(34) by salvaging available queuine.